{
  "gene_name": "Annexin A8-like protein 1",
  "gene": "UniProtKB:Q5VT79",
  "gene_symbol": "ANXA8L1",
  "term_id": "GO:0001786",
  "term_label": "phosphatidylserine binding"
}